ATP generation from poly-ADP-D-ribose [GO:1990966] (biological process) References: PMID:27257257 Definition: The process of generating ATP in the nucleus from poly-ADP-D-ribose. Nuclear ATP generation is required for extensive chromatin remodeling events that are energy-consuming. Relationships: is a type of macromolecule metabolic process [GO:0043170]; is a type of ATP metabolic process [GO:0046034]